{
  "gene_name": "P2Y purinoceptor 2",
  "gene_symbol": "P2RY2",
  "term_id": "GO:0005886",
  "term_label": "plasma membrane",
  "gene": "UniProtKB:P41231"
}